{
  "gene_name": "Collagen alpha-2(VIII) chain",
  "term_id": "GO:0031012",
  "term_label": "extracellular matrix",
  "gene_symbol": "COL8A2",
  "gene": "UniProtKB:P25067"
}